{
  "gene_symbol": "FAM168A",
  "gene_name": "Protein FAM168A",
  "term_id": "GO:1905053",
  "term_label": "positive regulation of base-excision repair",
  "gene": "UniProtKB:Q92567"
}